{
  "gene_name": "Zinc finger CCHC domain-containing protein 14",
  "gene_symbol": "ZCCHC14",
  "term_label": "Unknown cellular component",
  "gene": "UniProtKB:Q8WYQ9",
  "term_id": "UNKNOWN:0003"
}